{
  "gene_name": "Splicing regulator SDE2",
  "term_id": "UNKNOWN:0002",
  "gene_symbol": "SDE2",
  "term_label": "Unknown biological process",
  "gene": "UniProtKB:Q6IQ49"
}